{
  "gene_name": "Histone lysine demethylase PHF8",
  "term_id": "UNKNOWN:0003",
  "term_label": "Unknown cellular component",
  "gene": "UniProtKB:Q9UPP1",
  "gene_symbol": "PHF8"
}